{
  "term_id": "GO:0036297",
  "term_label": "interstrand cross-link repair",
  "gene": "UniProtKB:Q9Y2M0",
  "gene_name": "Fanconi-associated nuclease 1",
  "gene_symbol": "FAN1"
}